hexose transmembrane transporter activity [GO:0015149] (molecular function) Sources: GOC:ai, GOC:mtg_transport, ISBN:0815340729 Definition: Enables the transfer of a hexose sugar, a monosaccharide with 6 carbon atoms, from one side of a membrane to the other. Relationships: is a type of GO:0015145; is part of hexose transmembrane transport [GO:0008645] Subtypes: GO:0005353, galactose transmembrane transporter activity [GO:0005354], GO:0008516, GO:0009679, fucose transmembrane transporter activity [GO:0015150], GO:0015153, mannose transmembrane transporter activity [GO:0015578], ABC-type D-allose transporter activity [GO:0015615], D-glucose transmembrane transporter activity [GO:0055056]